{
  "gene_name": "Zinc finger protein 781",
  "term_id": "UNKNOWN:0002",
  "gene": "UniProtKB:Q8N8C0",
  "term_label": "Unknown biological process",
  "gene_symbol": "ZNF781"
}